{
  "gene_symbol": "RAD52",
  "term_id": "GO:0005634",
  "gene": "UniProtKB:P43351",
  "term_label": "nucleus",
  "gene_name": "DNA repair protein RAD52 homolog"
}